SCF-Rcy1/Pof6 ubiquitin ligase complex [GO:0097667] (cellular component) Relationships: is a type of SCF ubiquitin ligase complex [GO:0019005] Definition: An SCF ubiquitin ligase complex in which the F-box protein is Rcy1 in S. cerevisiae (Pof6 in S. pombe). References: PMID:14747994, PMID:15147268 Sources: GOC:jd, GOC:vw